{
  "gene_symbol": "ENTREP2",
  "gene": "UniProtKB:O60320",
  "gene_name": "Protein ENTREP2",
  "term_id": "UNKNOWN:0002",
  "term_label": "Unknown biological process"
}